{
  "gene": "UniProtKB:P23141",
  "term_label": "endoplasmic reticulum",
  "term_id": "GO:0005783",
  "gene_name": "Liver carboxylesterase 1",
  "gene_symbol": "CES1"
}